intercalated disc [GO:0014704] (cellular component) Relationships: is a type of cell-cell contact zone [GO:0044291] Also known as: intercalated disk Definition: A complex cell-cell junction at which myofibrils terminate in cardiomyocytes; mediates mechanical and electrochemical integration between individual cardiomyocytes. The intercalated disc contains regions of tight mechanical attachment (fasciae adherentes and desmosomes) and electrical coupling (gap junctions) between adjacent cells. References: PMID:11732910 Sources: GOC:mtg_muscle